{
  "gene_name": "Regulator of G-protein signaling 7",
  "term_id": "GO:0043005",
  "gene": "UniProtKB:P49802",
  "term_label": "neuron projection",
  "gene_symbol": "RGS7"
}